{
  "term_id": "GO:0043235",
  "gene": "UniProtKB:Q15303",
  "gene_name": "Receptor tyrosine-protein kinase erbB-4",
  "gene_symbol": "ERBB4",
  "term_label": "receptor complex"
}